{
  "term_id": "GO:0000209",
  "gene_name": "Kelch-like protein 42",
  "gene": "UniProtKB:Q9P2K6",
  "gene_symbol": "KLHL42",
  "term_label": "protein polyubiquitination"
}